microvillus organization [GO:0032528] (BP) Relationships: is a type of GO:0120036 Sources: GOC:mah Definition: A process that is carried out at the cellular level which results in the assembly, arrangement of constituent parts, or disassembly of a microvillus, a thin cylindrical membrane-covered projection on the surface of a cell. Also known as: microvillus organisation, microvillus organization and biogenesis Subtypes: microvillus assembly [GO:0030033], GO:0032529 Regulation: regulated by regulation of microvillus organization [GO:0032530]